{
  "term_label": "transcription factor TFIID complex",
  "gene_name": "TATA-box binding protein associated factor 11 like protein 2",
  "term_id": "GO:0005669",
  "gene_symbol": "TAF11L2",
  "gene": "UniProtKB:A6NLC8"
}